{
  "gene_symbol": "HOXA13",
  "gene": "UniProtKB:P31271",
  "term_label": "RNA polymerase II cis-regulatory region sequence-specific DNA binding",
  "gene_name": "Homeobox protein Hox-A13",
  "term_id": "GO:0000978"
}